regulation of epithelial cell proliferation involved in lung morphogenesis [GO:2000794] (biological process) Subtypes: GO:0060501, negative regulation of epithelial cell proliferation involved in lung morphogenesis [GO:2000795] References: PMID:21513708 Definition: Any process that modulates the frequency, rate or extent of epithelial cell proliferation involved in lung morphogenesis. Relationships: is a type of regulation of epithelial cell proliferation [GO:0050678]; RO_0002211 epithelial cell proliferation involved in lung morphogenesis [GO:0060502]